{
  "term_id": "UNKNOWN:0003",
  "gene_symbol": "NUDT13",
  "gene": "UniProtKB:Q86X67",
  "term_label": "Unknown cellular component",
  "gene_name": "NAD(P)H pyrophosphatase NUDT13, mitochondrial"
}